{
  "gene_symbol": "IGF2R",
  "gene_name": "Cation-independent mannose-6-phosphate receptor",
  "term_label": "protein targeting to lysosome",
  "gene": "UniProtKB:P11717",
  "term_id": "GO:0006622"
}